{
  "gene": "UniProtKB:O95747",
  "term_id": "GO:0035556",
  "gene_name": "Serine_threonine-protein kinase OSR1",
  "term_label": "intracellular signal transduction",
  "gene_symbol": "OXSR1"
}